blood coagulation, extrinsic pathway [GO:0007598] (biological process) Definition: A protein activation cascade that initiates blood coagulation, starting with a signal from tissue factor (TF), a cell-surface, integral-membrane protein, which converts Factor IX to IXa, and Factor IXa converts Factor X to Xa. Factor Xa then initiates the common pathway. Relationships: is a type of protein activation cascade [GO:0072376]; is part of blood coagulation, fibrin clot formation [GO:0072378] References: PMID:26018600 Sources: GOC:add, GOC:mah, GOC:pde Regulation: regulated by GO:2000263; negatively regulated by negative regulation of blood coagulation, extrinsic pathway [GO:2000264]; positively regulated by positive regulation of blood coagulation, extrinsic pathway [GO:2000265] Also known as: initiation of blood coagulation cascade, tissue factor pathway Note: See also the biological process term 'blood coagulation, intrinsic pathway ; GO:0007597' and 'blood coagulation, common pathway ; GO:0072377'.